{
  "gene_name": "Lysophosphatidic acid receptor 2",
  "term_label": "G protein-coupled receptor activity",
  "gene_symbol": "LPAR2",
  "term_id": "GO:0004930",
  "gene": "UniProtKB:Q9HBW0"
}